{
  "gene_symbol": "CTSO",
  "gene_name": "Cathepsin O",
  "gene": "UniProtKB:P43234",
  "term_id": "GO:0051603",
  "term_label": "proteolysis involved in protein catabolic process"
}